ventricular cardiac muscle cell development [GO:0055015] (biological process) Definition: The process whose specific outcome is the progression of a ventricular cardiac muscle cell over time, from its formation to the mature state. Cardiac muscle cells are striated muscle cells that are responsible for heart contraction. The ventricle is the part of the heart that pumps blood out of the organ. Sources: GOC:devbiol, GOC:mtg_muscle Also known as: ventricular cardiomyocyte development, ventricular heart muscle cell development Relationships: is a type of cardiac muscle cell development [GO:0055013]; is part of ventricular cardiac muscle cell differentiation [GO:0055012]